{
  "term_id": "UNKNOWN:0002",
  "gene_name": "Paraneoplastic antigen Ma2",
  "term_label": "Unknown biological process",
  "gene_symbol": "PNMA2",
  "gene": "UniProtKB:Q9UL42"
}